{
  "gene": "UniProtKB:Q15386",
  "term_id": "GO:0006511",
  "gene_name": "Ubiquitin-protein ligase E3C",
  "gene_symbol": "UBE3C",
  "term_label": "ubiquitin-dependent protein catabolic process"
}